{
  "gene_symbol": "P2RX3",
  "gene_name": "P2X purinoceptor 3",
  "term_id": "GO:0004931",
  "term_label": "extracellularly ATP-gated monoatomic cation channel activity",
  "gene": "UniProtKB:P56373"
}